{
  "term_label": "DNA-binding transcription factor activity, RNA polymerase II-specific",
  "gene_name": "Zinc finger protein 791",
  "gene_symbol": "ZNF791",
  "term_id": "GO:0000981",
  "gene": "UniProtKB:Q3KP31"
}